{
  "term_id": "GO:0061640",
  "gene_symbol": "SEPTIN14",
  "term_label": "cytoskeleton-dependent cytokinesis",
  "gene": "UniProtKB:Q6ZU15",
  "gene_name": "Septin-14"
}